negative regulation of gastrin-induced gastric acid secretion [GO:1903640] (biological process) Definition: Any process that stops, prevents or reduces the frequency, rate or extent of gastrin-induced gastric acid secretion. References: PMID:11123201 Sources: GOC:TermGenie, GO_REF:0000058 Relationships: is a type of negative regulation of gastric acid secretion [GO:0060455]; is a type of regulation of gastrin-induced gastric acid secretion [GO:1903639]; negatively regulates gastrin-induced gastric acid secretion [GO:0001698] Also known as: down regulation of gastrin-induced gastric acid secretion, down-regulation of gastrin-induced gastric acid secretion, downregulation of gastrin-induced gastric acid secretion, inhibition of gastrin-induced gastric acid secretion